induced systemic resistance [GO:0009682] (biological process) References: PMID:10234273, PMID:15233292, PMID:23386685 Relationships: is a type of defense response to bacterium [GO:0042742]; is a type of innate immune response [GO:0045087] Definition: A response to non-pathogenic bacteria that confers broad spectrum systemic resistance to disease that does not depend upon salicylic acid signaling.